{
  "term_label": "NADP binding",
  "gene_symbol": "PGD",
  "term_id": "GO:0050661",
  "gene": "UniProtKB:P52209",
  "gene_name": "6-phosphogluconate dehydrogenase, decarboxylating"
}